{
  "term_label": "90S preribosome",
  "gene_name": "Ribosomal RNA processing protein 36 homolog",
  "gene_symbol": "RRP36",
  "gene": "UniProtKB:Q96EU6",
  "term_id": "GO:0030686"
}